{
  "gene_symbol": "GLIPR1",
  "gene": "UniProtKB:P48060",
  "gene_name": "Glioma pathogenesis-related protein 1",
  "term_id": "GO:0005615",
  "term_label": "extracellular space"
}